kinesin complex [GO:0005871] (cellular component) Definition: Any complex that includes a dimer of molecules from the kinesin superfamily, a group of related proteins that contain an extended region of predicted alpha-helical coiled coil in the main chain that likely produces dimerization. The native complexes of several kinesin family members have also been shown to contain additional peptides, often designated light chains as all of the noncatalytic subunits that are currently known are smaller than the chain that contains the motor unit. Kinesin complexes generally possess a force-generating enzymatic activity, or motor, which converts the free energy of the gamma phosphate bond of ATP into mechanical work. References: PMID:32842864 Sources: GOC:mah Subtypes: GO:0005872, GO:0005873, GO:0016938, kinesin II complex [GO:0016939] Relationships: is_a GO:0005875